{
  "term_id": "GO:0005525",
  "gene_symbol": "TUBB4A",
  "term_label": "GTP binding",
  "gene": "UniProtKB:P04350",
  "gene_name": "Tubulin beta-4A chain"
}